protein kinase C signaling [GO:0070528] (biological process) Definition: A series of reactions, mediated by the intracellular serine/threonine kinase protein kinase C, which occurs as a result of a single trigger reaction or compound. Also known as: PKC signal transduction, protein kinase C signal transduction, PKC signaling cascade, protein kinase C signaling cascade, protein kinase C signalling cascade Regulation: regulated by regulation of protein kinase C signaling [GO:0090036]; positively regulated by positive regulation of protein kinase C signaling [GO:0090037]; negatively regulated by negative regulation of protein kinase C signaling [GO:0090038] Sources: GOC:BHF, GOC:mah Relationships: is a type of intracellular signal transduction [GO:0035556]